{
  "gene": "UniProtKB:P62308",
  "term_label": "SMN-Sm protein complex",
  "gene_name": "Small nuclear ribonucleoprotein G",
  "gene_symbol": "SNRPG",
  "term_id": "GO:0034719"
}